{
  "term_id": "GO:0005794",
  "gene_symbol": "RNF148",
  "gene": "UniProtKB:Q8N7C7",
  "term_label": "Golgi apparatus",
  "gene_name": "RING finger protein 148"
}